{
  "gene": "UniProtKB:Q9Y2P4",
  "gene_name": "Long-chain fatty acid transport protein 6",
  "term_label": "long-chain fatty acid import into cell",
  "gene_symbol": "SLC27A6",
  "term_id": "GO:0044539"
}